{
  "term_label": "DNA-binding transcription factor activity, RNA polymerase II-specific",
  "gene": "UniProtKB:A8MUV8",
  "gene_name": "Putative zinc finger protein 727",
  "term_id": "GO:0000981",
  "gene_symbol": "ZNF727"
}